{
  "gene_name": "Nucleoside diphosphate kinase A",
  "term_label": "Unknown biological process",
  "gene_symbol": "NME1",
  "gene": "UniProtKB:P15531",
  "term_id": "UNKNOWN:0002"
}